fumarate hydratase activity [GO:0004333] (MF) Definition: Catalysis of the reaction: (S)-malate = fumarate + H2O. Relationships: is a type of GO:0016836 Sources: EC:4.2.1.2, RHEA:12460 Also known as: (S)-malate hydro-lyase (fumarate-forming), (S)-malate hydro-lyase activity, L-malate hydro-lyase activity, fumarase activity